{
  "term_id": "UNKNOWN:0003",
  "gene_symbol": "RNF224",
  "gene": "UniProtKB:P0DH78",
  "gene_name": "RING finger protein 224",
  "term_label": "Unknown cellular component"
}